{
  "gene_symbol": "TGFBR1",
  "gene": "UniProtKB:P36897",
  "gene_name": "TGF-beta receptor type-1",
  "term_id": "GO:0016361",
  "term_label": "activin receptor activity, type I"
}